{
  "gene": "UniProtKB:Q9H7E2",
  "term_id": "GO:0003723",
  "gene_symbol": "TDRD3",
  "gene_name": "Tudor domain-containing protein 3",
  "term_label": "RNA binding"
}